{
  "gene_name": "Proteasome subunit beta type-3",
  "gene": "UniProtKB:P49720",
  "gene_symbol": "PSMB3",
  "term_id": "GO:0005829",
  "term_label": "cytosol"
}